proprioception involved in equilibrioception [GO:0051355] (biological process) Relationships: is a type of proprioception [GO:0019230]; is part of equilibrioception [GO:0050957] Definition: The series of events contributing to equilibrioception by which an organism senses the position, location, orientation, and movement of the body and its parts. Proprioception plays an important role in the ability of an organism to perceive its orientation with respect to gravity. Sources: GOC:ai Also known as: equilibrioception by proprioception, perception of orientation with respect to gravity by proprioception, proprioception during equilibrioception